{
  "gene_name": "Unconventional myosin-Ib",
  "gene": "UniProtKB:O43795",
  "term_label": "plasma membrane",
  "gene_symbol": "MYO1B",
  "term_id": "GO:0005886"
}